glycerol transmembrane transport [GO:0015793] (biological process) Definition: The directed movement of glycerol across a membrane. Glycerol is 1,2,3-propanetriol, a sweet, hygroscopic, viscous liquid, widely distributed in nature as a constituent of many lipids. Sources: GOC:ai Also known as: glycerol transport Relationships: is a type of polyol transmembrane transport [GO:0015791]; is a type of GO:0034219 Regulation: regulated by regulation of glycerol transport [GO:0090371]; positively regulated by positive regulation of glycerol transport [GO:0090372]; negatively regulated by GO:0090373